{
  "gene_symbol": "PDE3A",
  "term_label": "3',5'-cyclic-GMP phosphodiesterase activity",
  "gene": "UniProtKB:Q14432",
  "gene_name": "cGMP-inhibited 3',5'-cyclic phosphodiesterase 3A",
  "term_id": "GO:0047555"
}